regulation of granulosa cell apoptotic process [GO:1904708] (biological process) Also known as: regulation of granulosa cell of ovary apoptotic process, regulation of granulosa cell apoptosis, regulation of granulosa cell of ovary apoptosis References: PMID:19208546 Sources: GOC:TermGenie, GO_REF:0000058 Subtypes: negative regulation of granulosa cell apoptotic process [GO:1904709], positive regulation of granulosa cell apoptotic process [GO:1904710] Relationships: is a type of GO:1904035; regulates granulosa cell apoptotic process [GO:1904700] Definition: Any process that modulates the frequency, rate or extent of granulosa cell apoptotic process.